{
  "gene_symbol": "SCARA3",
  "term_id": "UNKNOWN:0002",
  "term_label": "Unknown biological process",
  "gene_name": "Scavenger receptor class A member 3",
  "gene": "UniProtKB:Q6AZY7"
}